{
  "term_id": "GO:0055001",
  "gene_symbol": "ACTN3",
  "gene": "UniProtKB:Q08043",
  "gene_name": "Alpha-actinin-3",
  "term_label": "muscle cell development"
}